{
  "term_id": "GO:0006955",
  "gene_symbol": "MARCHF1",
  "gene": "UniProtKB:Q8TCQ1",
  "gene_name": "E3 ubiquitin-protein ligase MARCHF1",
  "term_label": "immune response"
}